calcium ion transport from cytosol to endoplasmic reticulum [GO:1903515] (biological process) References: PMID:16402920 Sources: GOC:BHF, GOC:TermGenie, GOC:mtg_cardiac_conduct_nov11, GOC:rl, GO_REF:0000078 Relationships: is a type of cytosol to endoplasmic reticulum transport [GO:0046967]; is a type of calcium ion transmembrane transport [GO:0070588] Definition: The directed movement of calcium ion from cytosol to endoplasmic reticulum.